translational readthrough [GO:0006451] (biological process) Also known as: natural nonsense suppression Definition: The continuation of translation beyond a stop codon by the use of a special tRNA that recognizes the UAG and UGA codons as modified amino acids, rather than as termination codons. Relationships: is a type of GO:0006414; is_a GO:0006417 Subtypes: selenocysteine incorporation [GO:0001514], GO:0030631, viral translational readthrough [GO:0039705] References: PMID:11179232 Sources: GOC:jsg